{
  "gene_symbol": "TJP1",
  "gene_name": "Tight junction protein ZO-1",
  "gene": "UniProtKB:Q07157",
  "term_id": "GO:0098609",
  "term_label": "cell-cell adhesion"
}